{
  "gene": "UniProtKB:P29803",
  "term_id": "GO:0004739",
  "gene_symbol": "PDHA2",
  "gene_name": "Pyruvate dehydrogenase E1 component subunit alpha, testis-specific form, mitochondrial",
  "term_label": "pyruvate dehydrogenase (acetyl-transferring) activity"
}